{
  "term_id": "GO:0005634",
  "gene_name": "Zinc finger protein 674",
  "gene": "UniProtKB:Q2M3X9",
  "gene_symbol": "ZNF674",
  "term_label": "nucleus"
}